presynaptic density [GO:0098980] (cellular component) Subtypes: T-bar [GO:0098986] Relationships: is a type of GO:0048788 References: PMID:26780543 Sources: GOC:dos Definition: An electron dense specialization of the presynaptic active zone cytoskeleton.